flavonol-3-O-glycoside glucosyltransferase activity [GO:0033839] (MF) Sources: EC:2.4.1.240 Also known as: UDP-glucose:flavonol-3-O-beta-D-glucosyl-(1->2)-beta-D-glucoside 2'''-O-beta-D-glucosyltransferase activity Relationships: is a type of glucosyltransferase activity [GO:0046527] Definition: Catalysis of the reaction: UDP-glucose + a flavonol 3-O-beta-D-glucosyl-(1->2)-beta-D-glucoside = UDP + a flavonol 3-O-beta-D-glucosyl-(1->2)-beta-D-glucosyl-(1->2)-beta-D-glucoside.